{
  "term_label": "chromocenter",
  "gene_symbol": "MBD5",
  "gene_name": "Methyl-CpG-binding domain protein 5",
  "gene": "UniProtKB:Q9P267",
  "term_id": "GO:0010369"
}